{
  "gene_name": "F-box only protein 44",
  "term_id": "GO:0006516",
  "gene": "UniProtKB:Q9H4M3",
  "term_label": "glycoprotein catabolic process",
  "gene_symbol": "FBXO44"
}